toxin biosynthetic process [GO:0009403] (biological process) Sources: GOC:go_curators Also known as: toxin anabolism, toxin biosynthesis, toxin formation, toxin synthesis Relationships: is a type of toxin metabolic process [GO:0009404]; is_a secondary metabolite biosynthetic process [GO:0044550] Definition: The chemical reactions and pathways resulting in the formation of toxin, a poisonous compound (typically a protein) that is produced by cells or organisms and that can cause disease when introduced into the body or tissues of an organism. Subtypes: bacteriocin biosynthetic process [GO:0030152], mycotoxin biosynthetic process [GO:0043386], sterigmatocystin biosynthetic process [GO:0045461], GO:0052315